{
  "term_label": "minus-end-directed microtubule motor activity",
  "gene_symbol": "DNAH7",
  "term_id": "GO:0008569",
  "gene": "UniProtKB:Q8WXX0",
  "gene_name": "Dynein axonemal heavy chain 7"
}